{
  "gene_name": "Serine_threonine-protein kinase_endoribonuclease IRE2",
  "gene_symbol": "ERN2",
  "term_id": "GO:0004521",
  "gene": "UniProtKB:Q76MJ5",
  "term_label": "RNA endonuclease activity"
}